magnesium ion transport from cytosol to endoplasmic reticulum [GO:0160176] (biological process) Relationships: is a type of cytosol to endoplasmic reticulum transport [GO:0046967]; is a type of magnesium ion transmembrane transport [GO:1903830] Definition: The directed movement of magnesium ion from cytosol to endoplasmic reticulum. References: PMID:38513662